{
  "term_id": "GO:0005829",
  "term_label": "cytosol",
  "gene_name": "Ras association domain-containing protein 9",
  "gene_symbol": "RASSF9",
  "gene": "UniProtKB:O75901"
}